{
  "gene_name": "Thrombospondin-4",
  "term_label": "extracellular matrix",
  "gene_symbol": "THBS4",
  "term_id": "GO:0031012",
  "gene": "UniProtKB:P35443"
}